{
  "gene_name": "General transcription factor IIF subunit 1",
  "gene_symbol": "GTF2F1",
  "term_id": "GO:0005674",
  "gene": "UniProtKB:P35269",
  "term_label": "transcription factor TFIIF complex"
}